{
  "gene_name": "Ski-like protein",
  "term_id": "GO:0000122",
  "gene": "UniProtKB:P12757",
  "term_label": "negative regulation of transcription by RNA polymerase II",
  "gene_symbol": "SKIL"
}